{
  "gene": "UniProtKB:Q9NUE0",
  "term_id": "GO:0006612",
  "gene_symbol": "ZDHHC18",
  "gene_name": "Palmitoyltransferase ZDHHC18",
  "term_label": "protein targeting to membrane"
}